{
  "term_id": "GO:0004672",
  "gene": "UniProtKB:A0A087WV53",
  "gene_name": "SPEG neighbor protein",
  "gene_symbol": "SPEGNB",
  "term_label": "protein kinase activity"
}